{
  "gene_name": "cGMP-dependent 3',5'-cyclic phosphodiesterase",
  "term_id": "GO:0010628",
  "term_label": "positive regulation of gene expression",
  "gene_symbol": "PDE2A",
  "gene": "UniProtKB:O00408"
}